{
  "term_label": "receptor complex",
  "gene_name": "Leptin receptor",
  "gene_symbol": "LEPR",
  "term_id": "GO:0043235",
  "gene": "UniProtKB:P48357"
}